{
  "term_id": "UNKNOWN:0001",
  "gene": "UniProtKB:Q9NWS1",
  "gene_symbol": "PARPBP",
  "gene_name": "PCNA-interacting partner",
  "term_label": "Unknown molecular function"
}